{
  "gene_symbol": "EXOC5",
  "gene_name": "Exocyst complex component 5",
  "term_id": "GO:0000145",
  "gene": "UniProtKB:O00471",
  "term_label": "exocyst"
}